{
  "term_id": "GO:0007030",
  "gene_name": "Golgin subfamily A member 8S",
  "gene": "UniProtKB:H3BPF8",
  "gene_symbol": "GOLGA8S",
  "term_label": "Golgi organization"
}